{
  "term_id": "GO:0001228",
  "gene": "UniProtKB:Q9H161",
  "gene_symbol": "ALX4",
  "term_label": "DNA-binding transcription activator activity, RNA polymerase II-specific",
  "gene_name": "Homeobox protein aristaless-like 4"
}